oxytetracycline biosynthetic process [GO:1901763] (biological process) Definition: The chemical reactions and pathways resulting in the formation of oxytetracycline. Relationships: is a type of polyketide biosynthetic process [GO:0030639] Also known as: oxytetracycline anabolism, oxytetracycline biosynthesis, oxytetracycline formation, oxytetracycline synthesis References: PMID:8163168 Sources: GOC:TermGenie, GOC:yaf, UniPathway:UPA00926